endonucleolytic cleavage of tetracistronic rRNA transcript (SSU-rRNA, LSU-rRNA, 4.5S-rRNA, 5S-rRNA) [GO:0002103] (biological process) Definition: Endonucleolytic cleavage of a pre-rRNA molecule originally produced as a tetracistronic rRNA transcript that contains the Small Subunit (SSU) rRNA, Large Subunit (LSU) the 4.5S rRNA, and the 5S rRNA in that order from 5' to 3' along the primary transcript. Primary ribosomal RNA transcripts with four genes, in this order, are produced in the chloroplasts of vascular plants. Note that the use of the word tetracistronic refers only to the number of mature rRNA molecules which will be produced from the primary transcript and ignores tRNAs that may also be present within the primary transcript. Subtypes: endonucleolytic cleaveage between 4.5S rRNA and 5S rRNA of tetracistronic rRNA transcript (SSU-rRNA, LSU-rRNA, 4.5S-rRNA, 5S-rRNA) [GO:0002104], GO:0002105, GO:0002106 Relationships: is a type of rRNA processing [GO:0006364] Sources: GOC:curators